{
  "gene_name": "Modulator of apoptosis 1",
  "term_id": "UNKNOWN:0001",
  "term_label": "Unknown molecular function",
  "gene": "UniProtKB:Q96BY2",
  "gene_symbol": "MOAP1"
}